regulation of catecholamine metabolic process [GO:0042069] (biological process) Subtypes: regulation of dopamine metabolic process [GO:0042053] Relationships: is a type of regulation of amine metabolic process [GO:0033238]; is a type of regulation of primary metabolic process [GO:0080090]; regulates GO:0006584 Definition: Any process that modulates the frequency, rate or extent of the chemical reactions and pathways involving catecholamines. Also known as: regulation of catecholamine metabolism Sources: GOC:go_curators